{
  "term_label": "protein serine/threonine kinase activator activity",
  "term_id": "GO:0043539",
  "gene": "UniProtKB:Q2NL67",
  "gene_name": "Protein mono-ADP-ribosyltransferase PARP6",
  "gene_symbol": "PARP6"
}